positive regulation of transforming growth factor beta2 production [GO:0032915] (biological process) Definition: Any process that activates or increases the frequency, rate, or extent of production of transforming growth factor-beta2. Also known as: positive regulation of TGF-B2 production, positive regulation of TGFB2 production, positive regulation of transforming growth factor-beta2 production, up regulation of transforming growth factor-beta2 production, up-regulation of transforming growth factor-beta2 production, upregulation of transforming growth factor-beta2 production, activation of transforming growth factor-beta2 production, stimulation of transforming growth factor-beta2 production Sources: GOC:mah Relationships: is a type of regulation of transforming growth factor beta2 production [GO:0032909]; is a type of GO:0071636; positively regulates transforming growth factor beta2 production [GO:0032906]